{
  "gene": "UniProtKB:Q14974",
  "gene_name": "Importin subunit beta-1",
  "term_id": "GO:0006606",
  "term_label": "protein import into nucleus",
  "gene_symbol": "KPNB1"
}